allantoin biosynthetic process [GO:0019428] (biological process) Relationships: is a type of allantoin metabolic process [GO:0000255]; is a type of amide biosynthetic process [GO:0043604] Sources: GOC:go_curators Definition: The chemical reactions and pathways resulting in the formation of allantoin, (2,5-dioxo-4-imidazolidinyl)urea. Also known as: allantoin anabolism, allantoin biosynthesis, allantoin formation, allantoin synthesis